23S rRNA (adenine(2030)-N(6))-methyltransferase activity [GO:0036307] (molecular function) Definition: Catalysis of the reaction: S-adenosyl-L-methionine + adenine(2030) in 23S rRNA = S-adenosyl-L-homocysteine + rRNA containing N(6)-methyladenine(2030) in 23S rRNA. Relationships: is a type of rRNA (adenine-N6-)-methyltransferase activity [GO:0008988] References: PMID:22847818 Sources: GOC:imk, RHEA:43736